{
  "gene": "UniProtKB:Q3SYC2",
  "term_label": "endoplasmic reticulum membrane",
  "gene_name": "2-acylglycerol O-acyltransferase 2",
  "term_id": "GO:0005789",
  "gene_symbol": "MOGAT2"
}